cytokinin 7-beta-glucosyltransferase activity [GO:0047807] (molecular function) Also known as: cytokinin 7-b-glucosyltransferase activity, UDP-glucose-zeatin 7-glucosyltransferase activity, UDP-glucose:zeatin 7-glucosyltransferase activity, UDPglucose:zeatin 7-glucosyltransferase activity, cytokinin 7-glucosyltransferase activity, uridine diphosphoglucose-zeatin 7-glucosyltransferase activity Sources: EC:2.4.1.118, MetaCyc:CYTOKININ-7-BETA-GLUCOSYLTRANSFERASE-RXN Definition: Catalysis of the reaction: 6-alkylaminopurine + UDP-D-glucose = 6-alkylamino-7-beta-D-glucosylpurine + H+ + UDP. This reaction is an N-glucosylation event. Relationships: is a type of UDP-glucosyltransferase activity [GO:0035251]